{
  "gene_symbol": "GAR1",
  "term_label": "box H/ACA snoRNP complex",
  "gene": "UniProtKB:Q9NY12",
  "term_id": "GO:0031429",
  "gene_name": "H_ACA ribonucleoprotein complex subunit 1"
}